{
  "gene": "UniProtKB:Q15390",
  "gene_symbol": "MTFR1",
  "term_id": "GO:0005739",
  "gene_name": "Mitochondrial fission regulator 1",
  "term_label": "mitochondrion"
}